{
  "gene_name": "Serine_threonine-protein kinase MRCK alpha",
  "gene": "UniProtKB:Q5VT25",
  "term_label": "actomyosin structure organization",
  "term_id": "GO:0031032",
  "gene_symbol": "CDC42BPA"
}